{
  "term_label": "Unknown molecular function",
  "term_id": "UNKNOWN:0001",
  "gene_name": "Putative cytochrome P450 family member 4F30",
  "gene_symbol": "CYP4F30P",
  "gene": "UniProtKB:Q9H0H9"
}